N8-acetylspermidine:oxygen oxidoreductase (propane-1,3-diamine-forming) activity [GO:0052897] (molecular function) Relationships: is a type of GO:0046592 Also known as: N(8)-acetylspermidine oxidase (propane-1,3-diamine-forming) activity Definition: Catalysis of the reaction: H2O + N(8)-acetylspermidine + O2 = 1,3-diaminopropane + 4-acetamidobutanal + H2O2. Also active with N(1)-acetylspermine, weak activity with N(1),N(12)- diacetylspermine. Sources: EC:1.5.3.15, RHEA:25972